fructoselysine catabolic process [GO:1901281] (biological process) Sources: GOC:TermGenie, GOC:yaf, UniPathway:UPA00784 Also known as: fructosyllysine breakdown, fructosyllysine catabolic process, fructosyllysine catabolism, fructosyllysine degradation Definition: The chemical reactions and pathways resulting in the breakdown of fructoselysine. Relationships: is a type of GO:0030392; is a type of fructoselysine metabolic process [GO:0030393]; is a type of carboxylic acid catabolic process [GO:0046395]